{
  "gene_symbol": "NUSAP1",
  "term_label": "mitotic chromosome condensation",
  "gene_name": "Nucleolar and spindle-associated protein 1",
  "gene": "UniProtKB:Q9BXS6",
  "term_id": "GO:0007076"
}